antigen sampling by dendritic cells in mucosal-associated lymphoid tissue [GO:0002405] (biological process) Definition: The process of antigen sampling carried out by dendritic cells in the mucosal-associated lymphoid tissue. References: PMID:11896763, PMID:15681746 Sources: GOC:jal Also known as: antigen sampling by dendritic cells in MALT Relationships: is a type of GO:0002404; is part of dendritic cell antigen processing and presentation [GO:0002468]